Ubisch body [GO:0070645] (cellular component) References: PMID:14612572, PMID:16524248 Sources: GOC:ecd, GOC:mah Definition: A small, granular structure that is found in the extracellular matrix of cell of the secretory tapetal layer that surrounds developing pollen grains. Ubisch bodies have a sporopollenin coat, are attached to the peritapetal wall, and may play a role in pollen development. Relationships: is a type of cellular anatomical structure [GO:0110165]; is part of specialized extracellular matrix [GO:0140047] Also known as: orbicule